steroid 17-alpha-monooxygenase activity [GO:0004508] (molecular function) Definition: Catalysis of the reaction: a C21-steroid + O2 + reduced [NADPH--hemoprotein reductase] = a 17alpha-hydroxy-C21-steroid + H+ + H2O + oxidized [NADPH--hemoprotein reductase]. Relationships: is a type of GO:0008395; is a type of oxidoreductase activity, acting on paired donors, with incorporation or reduction of molecular oxygen, reduced flavin or flavoprotein as one donor, and incorporation of one atom of oxygen [GO:0016712] Sources: RHEA:65760 Subtypes: GO:0047096 Also known as: steroid 17-alpha-hydroxylase activity, steroid 17-alpha-hydroxylase-C17-20 lyase activity, cytochrome P450 CYP17, cytochrome p450 XVIIA1 activity, 17alpha-hydroxylase-C17,20 lyase activity, cytochrome P-450 (P-45017alpha,lyase), cytochrome P45017alpha, steroid 17-alpha-hydroxylase/17,20 lyase activity, steroid 17alpha-hydroxylase activity, steroid 17alpha-monooxygenase activity, steroid 17alphahydroxylase/17,20 lyase activity, steroid,hydrogen-donor:oxygen oxidoreductase (17alpha-hydroxylating)